inositol-1,2,3,4,6-pentakisphosphate 5-kinase activity [GO:0102732] (molecular function) Relationships: is a type of inositol pentakisphosphate kinase activity [GO:0120517] Also known as: 1D-myo-inositol-pentakisphosphate 5-kinase activity, inositol-pentakisphosphate 5-kinase activity, 1D-myo-inositol-1,2,3,4,6-heptakisphosphate 5-kinase activity Definition: Catalysis of the reaction: 1D-myo-inositol 1,2,3,4,6-pentakisphosphate + ATP = 1D-myo-inositol hexakisphosphate + ADP + H+. References: PMID:12226109 Sources: MetaCyc:RXN-7186